positive regulation of long-chain fatty acid import across plasma membrane [GO:0010747] (biological process) Note: While there is not universal consensus on the lengths of short-, medium-, long- and very-long-chain fatty acids, the GO uses the definitions in ChEBI (see CHEBI:26666, CHEBI:59554, CHEBI:15904 and CHEBI:27283). Sources: GOC:BHF, GOC:dph, GOC:tb Definition: Any process that increases the rate, frequency or extent of plasma membrane long-chain fatty acid transport. Plasma membrane long-chain fatty acid transport is the directed movement of long-chain fatty acids across the plasma membrane. A long-chain fatty acid has an aliphatic tail containing 13 to 22 carbons. Also known as: positive regulation of plasma membrane long-chain fatty acid transport Relationships: is a type of GO:0010746; is a type of positive regulation of transmembrane transport [GO:0034764]; is a type of positive regulation of long-chain fatty acid import into cell [GO:0140214]; positively regulates long-chain fatty acid import across plasma membrane [GO:0015911]